one-carbon metabolic process [GO:0006730] (biological process) Also known as: one carbon metabolic process, one carbon metabolism, one-carbon metabolism, one-carbon transfer metabolic process, one-carbon transfer metabolism Sources: GOC:hjd, GOC:mah, GOC:pde Relationships: is a type of GO:0044281 Subtypes: serine-isocitrate lyase pathway [GO:0019496], GO:0035999 Definition: The chemical reactions and pathways involving the transfer of one-carbon units in various oxidation states.